{
  "gene": "UniProtKB:O95716",
  "term_id": "GO:0005886",
  "gene_symbol": "RAB3D",
  "gene_name": "Ras-related protein Rab-3D",
  "term_label": "plasma membrane"
}